R-SMAD binding [GO:0070412] (molecular function) Definition: Binding to a receptor-regulated SMAD signaling protein. Also known as: pathway restricted SMAD binding, pathway-restricted SMAD binding, receptor regulated SMAD binding, receptor-regulated SMAD binding References: PMID:19114992 Sources: GOC:BHF, GOC:vk Relationships: is a type of GO:0046332